{
  "gene": "UniProtKB:A6NCW7",
  "gene_name": "Inactive ubiquitin carboxyl-terminal hydrolase 17-like protein 4",
  "gene_symbol": "USP17L4",
  "term_id": "GO:0031647",
  "term_label": "regulation of protein stability"
}